{
  "gene_name": "Chordin",
  "gene_symbol": "CHRD",
  "term_id": "GO:0009953",
  "gene": "UniProtKB:Q9H2X0",
  "term_label": "dorsal/ventral pattern formation"
}